L-asparagine transmembrane transporter activity [GO:0015182] (molecular function) Also known as: L-asparagine transporter activity, asparagine/glutamine permease activity Definition: Enables the transfer of L-asparagine from one side of a membrane to the other. L-asparagine is the L-enantiomer of alpha-aminosuccinamic acid. Sources: GOC:go_curators, GOC:jsg, GOC:mah, GOC:mtg_transport, ISBN:0198506732 Relationships: is a type of neutral L-amino acid transmembrane transporter activity [GO:0015175]; is a type of L-amino acid transmembrane transporter activity [GO:0015179]; is a type of amide transmembrane transporter activity [GO:0042887]; is part of asparagine transport [GO:0006867] Subtypes: L-asparagine, sodium:proton antiporter activity [GO:0140831], L-asparagine:sodium symporter activity [GO:0140901]